negative regulation of metabolic activity involved in hibernation [GO:0044250] (biological process) Definition: The slowing of metabolic processes to very low levels in order to conserve energy as a part of hibernation. Also known as: inhibition of metabolic activity during hibernation, down regulation of metabolic activity during hibernation, down-regulation of metabolic activity during hibernation, downregulation of metabolic activity during hibernation, negative regulation of metabolic activity during hibernation Relationships: is a type of negative regulation of metabolic process [GO:0009892]; is part of GO:0042750 Sources: GOC:jl, Wikipedia:Hibernation